{
  "gene_name": "Immediate early response 3-interacting protein 1",
  "term_label": "Unknown molecular function",
  "term_id": "UNKNOWN:0001",
  "gene_symbol": "IER3IP1",
  "gene": "UniProtKB:Q9Y5U9"
}